{
  "term_id": "GO:0005634",
  "gene": "UniProtKB:Q96K76",
  "gene_symbol": "USP47",
  "gene_name": "Ubiquitin carboxyl-terminal hydrolase 47",
  "term_label": "nucleus"
}